{
  "gene": "UniProtKB:Q9Y446",
  "term_label": "cell-cell adhesion",
  "gene_name": "Plakophilin-3",
  "term_id": "GO:0098609",
  "gene_symbol": "PKP3"
}